{
  "gene": "UniProtKB:Q96SN8",
  "gene_symbol": "CDK5RAP2",
  "term_label": "chromosome segregation",
  "gene_name": "CDK5 regulatory subunit-associated protein 2",
  "term_id": "GO:0007059"
}